{
  "gene_name": "Lymphocyte activation gene 3 protein",
  "gene_symbol": "LAG3",
  "term_label": "transmembrane signaling receptor activity",
  "gene": "UniProtKB:P18627",
  "term_id": "GO:0004888"
}